fatty acid elongase complex [GO:0009923] (cellular component) Definition: A tetrameric complex of four different subunits which catalyzes the elongation of a fatty acid chain 2 carbon units at a time in the synthesis of very long chain fatty acids. Relationships: is a type of membrane protein complex [GO:0098796]; is a type of GO:0140534; is a type of GO:1990234; is part of endoplasmic reticulum membrane [GO:0005789] Sources: GOC:tb